{
  "gene": "UniProtKB:P55916",
  "gene_symbol": "UCP3",
  "term_label": "response to cold",
  "term_id": "GO:0009409",
  "gene_name": "Putative mitochondrial transporter UCP3"
}